{
  "gene_name": "Testis anion transporter 1",
  "term_id": "GO:0005886",
  "gene": "UniProtKB:Q96RN1",
  "term_label": "plasma membrane",
  "gene_symbol": "SLC26A8"
}